dinoflagellate apical horn [GO:0097686] (cellular component) References: PMID:7002229 Sources: GOC:at Definition: A horn-shaped dinoflagellate apex found in thecate species. Relationships: is a type of GO:0097683